{
  "term_label": "chaperonin-containing T-complex",
  "term_id": "GO:0005832",
  "gene_name": "T-complex protein 1 subunit gamma",
  "gene_symbol": "CCT3",
  "gene": "UniProtKB:P49368"
}